URM1 conjugating enzyme activity [GO:0061658] (molecular function) Sources: GOC:dph Relationships: is a type of URM1 transferase activity [GO:0042294]; is a type of GO:0061650 Definition: Isoenergetic transfer of URM1 from one protein to another via the reaction X-URM1 + Y = Y-URM1 + X, where both the X-URM1 and Y-URM1 linkages are thioester bonds between the C-terminal amino acid of URM1 and a sulfhydryl side group of a cysteine residue. Also known as: E2